endocytosed protein transport to vacuole [GO:0007038] (biological process) Relationships: is a type of intracellular protein transport [GO:0006886]; is a type of vacuolar transport [GO:0007034] Sources: GOC:ai Definition: The directed movement of proteins imported into a cell by endocytosis to the vacuole. Note: See also the biological process term 'endocytosis ; GO:0006897'. Also known as: delivery of endocytosed proteins to the vacuole